{
  "gene": "UniProtKB:Q8NB91",
  "gene_name": "Fanconi anemia group B protein",
  "term_label": "positive regulation of double-strand break repair via homologous recombination",
  "gene_symbol": "FANCB",
  "term_id": "GO:1905168"
}